{
  "gene_symbol": "RUBCNL",
  "term_id": "GO:0061910",
  "gene": "UniProtKB:Q9H714",
  "term_label": "autophagosome-endosome fusion",
  "gene_name": "Protein associated with UVRAG as autophagy enhancer"
}